{
  "term_id": "GO:0007416",
  "term_label": "synapse assembly",
  "gene": "UniProtKB:Q9ULL4",
  "gene_name": "Plexin-B3",
  "gene_symbol": "PLXNB3"
}